{
  "gene": "UniProtKB:Q9NQV6",
  "gene_symbol": "PRDM10",
  "term_label": "nucleus",
  "gene_name": "PR domain zinc finger protein 10",
  "term_id": "GO:0005634"
}